D-glucose:proton symporter activity [GO:0005356] (molecular function) Sources: GOC:mtg_transport Relationships: is a type of hexose:proton symporter activity [GO:0009679]; is a type of D-glucose transmembrane transporter activity [GO:0055056] Subtypes: high-affinity D-glucose:proton symporter activity [GO:0005358], low-affinity D-glucose:proton symporter activity [GO:0005359], insulin-responsive D-glucose:proton symporter activity [GO:0005360] Also known as: glucose:proton symporter activity, hydrogen:glucose symporter activity, transepithelial hydrogen:glucose symporter activity, hydrogen:glucose transporter activity, transepithelial hydrogen/glucose transporter activity, transepithelial hydrogen:glucose transporter activity Definition: Enables the transfer of a solute or solutes from one side of a membrane to the other according to the reaction: D-glucose + H+ = D-glucose + H+. Symporter activity enables the active transport of a solute across a membrane by a mechanism whereby two or more species are transported together in the same direction in a tightly coupled process not directly linked to a form of energy other than chemiosmotic energy.